{
  "gene_name": "Probable methyltransferase-like protein 25",
  "gene": "UniProtKB:Q8N6Q8",
  "term_label": "Unknown biological process",
  "term_id": "UNKNOWN:0002",
  "gene_symbol": "METTL25"
}